{
  "term_id": "GO:0008331",
  "term_label": "high voltage-gated calcium channel activity",
  "gene_name": "Voltage-dependent L-type calcium channel subunit beta-1",
  "gene_symbol": "CACNB1",
  "gene": "UniProtKB:Q02641"
}